{
  "gene_symbol": "USF1",
  "gene_name": "Upstream stimulatory factor 1",
  "gene": "UniProtKB:P22415",
  "term_label": "RNA polymerase II cis-regulatory region sequence-specific DNA binding",
  "term_id": "GO:0000978"
}